negative regulation of core promoter binding [GO:1904797] (biological process) Definition: Any process that stops, prevents or reduces the frequency, rate or extent of core promoter binding. Also known as: down regulation of core promoter binding, down-regulation of core promoter binding, downregulation of core promoter binding, inhibition of core promoter binding Relationships: is a type of negative regulation of transcription regulatory region DNA binding [GO:2000678]; negatively regulates GO:0001046 References: PMID:22723415 Sources: GOC:BHF, GOC:BHF_telomere, GOC:TermGenie, GOC:nc, GO_REF:0000059